{
  "gene": "UniProtKB:Q8WU58",
  "term_label": "Unknown molecular function",
  "gene_symbol": "FAM222B",
  "gene_name": "Protein FAM222B",
  "term_id": "UNKNOWN:0001"
}